{
  "gene": "UniProtKB:P63261",
  "term_id": "GO:0048870",
  "term_label": "cell motility",
  "gene_name": "Actin, cytoplasmic 2",
  "gene_symbol": "ACTG1"
}